{
  "gene_symbol": "CUL2",
  "gene": "UniProtKB:Q13617",
  "gene_name": "Cullin-2",
  "term_id": "GO:0031625",
  "term_label": "ubiquitin protein ligase binding"
}